{
  "term_id": "UNKNOWN:0002",
  "term_label": "Unknown biological process",
  "gene": "UniProtKB:P0DUQ2",
  "gene_name": "PRAME family member 9",
  "gene_symbol": "PRAMEF9"
}